intermembrane sphingolipid transfer [GO:0120012] (biological process) Relationships: is a type of GO:0071705; is_a intermembrane lipid transfer [GO:0120009] References: PMID:20823909, PMID:24220498, PMID:25797198 Sources: GOC:krc Definition: The transport of sphingolipids between membranes in which a sphingolipid molecule is transported through an aqueous phase from the outer leaflet of a donor membrane to the outer leaflet of an acceptor membrane. This process does not require metabolic energy and can be either spontaneous or mediated by lipid transfer proteins (LTPs).